adenosine nucleosidase activity [GO:0047622] (molecular function) Definition: Catalysis of the reaction: adenosine + H2O = D-ribose + adenine. Also known as: ANase activity, N-ribosyladenine ribohydrolase activity, adenosinase activity, adenosine hydrolase activity, adenosine ribohydrolase activity Relationships: is a type of purine nucleosidase activity [GO:0008477] Sources: EC:3.2.2.7, MetaCyc:ADENOSINE-NUCLEOSIDASE-RXN